renal albumin absorption [GO:0097018] (biological process) Regulation: regulated by regulation of renal albumin absorption [GO:2000532]; negatively regulated by GO:2000533; positively regulated by positive regulation of renal albumin absorption [GO:2000534] References: PMID:18431508 Sources: GOC:yaf Definition: A renal system process in which albumin is taken up from the collecting ducts, glomerulus and proximal and distal loops of the nephron. Relationships: is a type of renal protein absorption [GO:0097017]